positive regulation of lactation by mesenchymal-epithelial cell signaling [GO:0060637] (biological process) Also known as: positive regulation of lactation by mesenchymal-epithelial cell signalling Definition: The process that increases the rate, frequency, or extent of lactation as a result of the secretion of a signal from the mammary fat and its reception by a mammary epithelial cell. References: PMID:12558599 Sources: GOC:dph Relationships: is a type of mesenchymal-epithelial cell signaling [GO:0060638]; is a type of positive regulation of lactation [GO:1903489]